dynein complex [GO:0030286] (cellular component) Definition: Any of several large complexes that contain two or three dynein heavy chains and several light chains, and have microtubule motor activity. Relationships: is_a GO:0005875; is_a catalytic complex [GO:1902494] Sources: ISBN:0815316194 Subtypes: axonemal dynein complex [GO:0005858], cytoplasmic dynein complex [GO:0005868]